{
  "gene": "UniProtKB:P48146",
  "term_label": "neuropeptide binding",
  "term_id": "GO:0042923",
  "gene_name": "Neuropeptides B_W receptor type 2",
  "gene_symbol": "NPBWR2"
}